{
  "term_id": "GO:0008240",
  "gene_symbol": "TPP2",
  "gene": "UniProtKB:P29144",
  "gene_name": "Tripeptidyl-peptidase 2",
  "term_label": "tripeptidyl-peptidase activity"
}